nucleoside-specific channel forming porin activity [GO:0015471] (molecular function) Sources: GOC:mtg_transport Definition: Enables the energy independent passage of nucleoside, sized less than 1000 Da, across a membrane. The transmembrane portions of porins consist exclusively of beta-strands which form a beta-barrel. They are found in the outer membranes of Gram-negative bacteria, mitochondria, plastids and possibly acid-fast Gram-positive bacteria. Relationships: is a type of nucleoside transmembrane transporter activity [GO:0005337]; is a type of GO:0015288